{
  "term_id": "UNKNOWN:0003",
  "term_label": "Unknown cellular component",
  "gene_name": "G patch domain and ankyrin repeat-containing protein 1",
  "gene": "UniProtKB:O95872",
  "gene_symbol": "GPANK1"
}